retroviral intasome [GO:0044834] (cellular component) Relationships: is a type of protein-DNA complex [GO:0032993] Definition: A tetramer of retroviral integrase subunits tightly associated with a pair of viral DNA ends. Functions to insert viral DNA into a host cell chromosome. References: PMID:20118915